nucleotide-activated protein kinase complex [GO:0031588] (CC) Sources: GOC:bhm, GOC:mah, GOC:vw Definition: A protein complex that possesses nucleotide-dependent protein kinase activity. The nucleotide can be AMP (in S. pombe and human) or ADP (in S. cerevisiae). Relationships: is a type of GO:0140535; is a type of GO:1902911 Also known as: 5'-AMP-activated protein kinase complex, ADP-activated protein kinase complex, AMP-activated protein kinase complex, SNF1/AMPK protein kinase complex, Snf1 kinase complex, Snf1 serine/threonine protein kinase complex, AMPK complex